PSI associated light-harvesting complex I, LHCIa subcomplex [GO:0030083] (cellular component) Definition: A pigment protein complex that forms part of the photosystem I associated light-harvesting complex I; contains two proteins (usually about 24 and 21.5 kDa); has a fluorescence maximum between 680 and 690 nm. References: PMID:8825475 Relationships: is a type of PSI associated light-harvesting complex I [GO:0009518]